{
  "gene": "UniProtKB:Q9NPU4",
  "term_label": "Unknown molecular function",
  "gene_symbol": "C14orf132",
  "term_id": "UNKNOWN:0001",
  "gene_name": "Uncharacterized protein C14orf132"
}